ABC-type peptide transporter activity [GO:0015440] (molecular function) Subtypes: ABC-type peptide antigen transporter activity [GO:0015433] Sources: EC:7.4.2.5 Also known as: peptide ABC transporter, ATP-dependent peptide transmembrane transporter activity, ATPase-coupled peptide transmembrane transporter activity, peptide-transporting ATPase activity Definition: Catalysis of the reaction: ATP + H2O + peptide(in) = ADP + phosphate + peptide(out). Peptides exported include alpha-hemolysin, cyclolysin, colicin V and siderophores from Gram-negative bacteria, and bacteriocin, subtilin, competence factor and pediocin from Gram-positive bacteria. Relationships: is a type of ABC-type transporter activity [GO:0140359]; is a type of GO:1904680; is part of peptide transport [GO:0015833]